{
  "term_id": "GO:0005634",
  "gene_name": "Ubiquitin carboxyl-terminal hydrolase 17-like protein 11",
  "term_label": "nucleus",
  "gene": "UniProtKB:C9JVI0",
  "gene_symbol": "USP17L11"
}